{
  "term_id": "UNKNOWN:0001",
  "gene_name": "Glutathione S-transferase C-terminal domain-containing protein",
  "gene_symbol": "GSTCD",
  "gene": "UniProtKB:Q8NEC7",
  "term_label": "Unknown molecular function"
}